{
  "term_id": "UNKNOWN:0003",
  "gene_name": "POTE ankyrin domain family member C",
  "gene": "UniProtKB:B2RU33",
  "gene_symbol": "POTEC",
  "term_label": "Unknown cellular component"
}